camera-type eye development [GO:0043010] (biological process) Sources: GOC:go_curators, GOC:mtg_sensu Subtypes: embryonic camera-type eye development [GO:0031076], post-embryonic camera-type eye development [GO:0031077] Definition: The process whose specific outcome is the progression of the camera-type eye over time, from its formation to the mature structure. The camera-type eye is an organ of sight that receives light through an aperture and focuses it through a lens, projecting it on a photoreceptor field. Relationships: is a type of GO:0001654